malate:proton symporter activity [GO:0015366] (molecular function) Also known as: malate:hydrogen symporter activity, L-malic acid permease, L-malic acid:proton symporter activity, malate permease Relationships: is a type of GO:0015140; is a type of GO:0015295 Sources: TC:2.A.16.2.1 Definition: Enables the transfer of a solute or solutes from one side of a membrane to the other according to the reaction: malate(out) + H+(out) = malate(in) + H+(in).